{
  "gene_symbol": "NPPB",
  "term_label": "receptor guanylyl cyclase signaling pathway",
  "term_id": "GO:0007168",
  "gene_name": "Natriuretic peptides B",
  "gene": "UniProtKB:P16860"
}